{
  "gene_name": "Zinc finger protein 284",
  "term_label": "RNA polymerase II cis-regulatory region sequence-specific DNA binding",
  "term_id": "GO:0000978",
  "gene": "UniProtKB:Q2VY69",
  "gene_symbol": "ZNF284"
}